{
  "gene": "UniProtKB:Q8NGK2",
  "gene_name": "Olfactory receptor 52B4",
  "gene_symbol": "OR52B4",
  "term_label": "plasma membrane",
  "term_id": "GO:0005886"
}